{
  "gene_name": "Glucose-induced degradation protein 8 homolog",
  "term_id": "GO:0043161",
  "gene": "UniProtKB:Q9NWU2",
  "gene_symbol": "GID8",
  "term_label": "proteasome-mediated ubiquitin-dependent protein catabolic process"
}